regulation of endocannabinoid signaling pathway [GO:2000124] (biological process) References: PMID:15550444 Sources: GOC:mah Definition: Any process that modulates the frequency, rate or extent of endocannabinoid signaling pathway. Also known as: regulation of endocannabinoid signalling pathway Relationships: is a type of regulation of G protein-coupled receptor signaling pathway [GO:0008277]; RO_0002211 endocannabinoid signaling pathway [GO:0071926]